response to auditory stimulus [GO:0010996] (BP) Relationships: is a type of GO:0009612 Sources: GOC:BHF, GOC:dph, GOC:sl, GOC:tb Definition: Any process that results in a change in state or activity of a cell or an organism (in terms of movement, secretion, enzyme production, gene expression, etc.) as a result of an auditory stimulus. Also known as: response to sound, response to sound stimulus